{
  "term_id": "UNKNOWN:0001",
  "gene": "UniProtKB:Q96Q27",
  "gene_name": "Ankyrin repeat and SOCS box protein 2",
  "gene_symbol": "ASB2",
  "term_label": "Unknown molecular function"
}